{
  "term_id": "GO:0005737",
  "gene_name": "E3 ubiquitin-protein ligase RNF144B",
  "gene_symbol": "RNF144B",
  "gene": "UniProtKB:Q7Z419",
  "term_label": "cytoplasm"
}